{
  "gene_name": "Nuclear cap-binding protein subunit 2-like",
  "term_label": "nuclear cap binding complex",
  "gene": "UniProtKB:A6PVI3",
  "gene_symbol": "NCBP2L",
  "term_id": "GO:0005846"
}